synaptonemal complex assembly [GO:0007130] (biological process) Also known as: synaptonemal complex formation Relationships: is a type of cellular component assembly [GO:0022607]; is a type of GO:0070192; is a type of GO:0070193; is part of homologous chromosome pairing at meiosis [GO:0007129] Sources: ISBN:0198506732 Definition: The cell cycle process in which the synaptonemal complex is formed. This is a structure that holds paired chromosomes together during prophase I of meiosis and that promotes genetic recombination. Regulation: regulated by regulation of synaptonemal complex assembly [GO:0090173]; positively regulated by GO:1905088